{
  "term_label": "epigenetic regulation of gene expression",
  "gene_name": "Histone deacetylase 5",
  "term_id": "GO:0040029",
  "gene_symbol": "HDAC5",
  "gene": "UniProtKB:Q9UQL6"
}